{
  "gene": "UniProtKB:O15260",
  "term_label": "endoplasmic reticulum",
  "term_id": "GO:0005783",
  "gene_name": "Surfeit locus protein 4",
  "gene_symbol": "SURF4"
}